{
  "term_label": "nucleus",
  "gene_symbol": "MCM8",
  "gene": "UniProtKB:Q9UJA3",
  "term_id": "GO:0005634",
  "gene_name": "DNA helicase MCM8"
}